positive regulation of coenzyme F420-dependent bicyclic nitroimidazole catabolic process [GO:1900290] (biological process) Sources: GOC:TermGenie, GOC:mengo_curators Also known as: positive regulation of coenzyme F420-dependent nitroimidazole breakdown, positive regulation of coenzyme F420-dependent nitroimidazole catabolism, positive regulation of coenzyme F420-dependent nitroimidazole reduction, up regulation of coenzyme F420-dependent bicyclic nitroimidazole catabolic process, up regulation of coenzyme F420-dependent nitroimidazole breakdown, up regulation of coenzyme F420-dependent nitroimidazole catabolism, up regulation of coenzyme F420-dependent nitroimidazole reduction, up-regulation of coenzyme F420-dependent bicyclic nitroimidazole catabolic process, up-regulation of coenzyme F420-dependent nitroimidazole breakdown, up-regulation of coenzyme F420-dependent nitroimidazole catabolism, up-regulation of coenzyme F420-dependent nitroimidazole reduction, upregulation of coenzyme F420-dependent bicyclic nitroimidazole catabolic process, upregulation of coenzyme F420-dependent nitroimidazole breakdown, upregulation of coenzyme F420-dependent nitroimidazole catabolism, upregulation of coenzyme F420-dependent nitroimidazole reduction, activation of coenzyme F420-dependent bicyclic nitroimidazole catabolic process, activation of coenzyme F420-dependent nitroimidazole breakdown, activation of coenzyme F420-dependent nitroimidazole catabolism, activation of coenzyme F420-dependent nitroimidazole reduction, activation of coenzyme F420-dependent nitroreductase activity, positive regulation of coenzyme F420-dependent nitroreductase activity, up regulation of coenzyme F420-dependent nitroreductase activity, up-regulation of coenzyme F420-dependent nitroreductase activity, upregulation of coenzyme F420-dependent nitroreductase activity Definition: Any process that activates or increases the frequency, rate or extent of coenzyme F420-dependent bicyclic nitroimidazole catabolic process. Relationships: is a type of GO:0009896; is a type of regulation of coenzyme F420-dependent bicyclic nitroimidazole catabolic process [GO:1900288]; positively regulates coenzyme F420-dependent bicyclic nitroimidazole catabolic process [GO:0052799]